negative regulation of phagosome maturation [GO:1905163] (biological process) Also known as: down regulation of phagosome maturation, down-regulation of phagosome maturation, downregulation of phagosome maturation, inhibition of phagosome maturation Relationships: is a type of negative regulation of organelle organization [GO:0010639]; is a type of GO:1905162; negatively regulates phagosome maturation [GO:0090382] Definition: Any process that stops, prevents or reduces the frequency, rate or extent of phagosome maturation. Sources: GOC:PARL, GOC:TermGenie, GOC:bf, GO_REF:0000058